{
  "gene_name": "fMet-Leu-Phe receptor",
  "term_id": "GO:0007204",
  "term_label": "positive regulation of cytosolic calcium ion concentration",
  "gene_symbol": "FPR1",
  "gene": "UniProtKB:P21462"
}